{
  "gene": "UniProtKB:P62312",
  "term_id": "GO:0005732",
  "term_label": "sno(s)RNA-containing ribonucleoprotein complex",
  "gene_symbol": "LSM6",
  "gene_name": "U6 snRNA-associated Sm-like protein LSm6"
}